antigen processing and presentation of endogenous peptide antigen via MHC class I via ER pathway, TAP-dependent [GO:0002485] (biological process) Definition: The process in which an antigen-presenting cell expresses a peptide antigen of endogenous origin on its cell surface in association with an MHC class I protein complex following intracellular transport via a TAP-dependent ER pathway. The peptide is typically a fragment of a larger endogenous protein which has been degraded within the cell and becomes associated with the MHC class I molecule in the ER following TAP-dependent transport from the cytosol. Class I here refers to classical class I molecules. Also known as: TAP-dependent antigen processing and presentation of endogenous peptide antigen via MHC class I via ER pathway, TAP-dependent endogenous peptide antigen processing and presentation via MHC class I via ER pathway, endogenous peptide antigen processing and presentation via MHC class I via ER pathway, TAP-dependent References: PMID:14647477, PMID:15771591 Sources: GOC:add, ISBN:0781735149 Relationships: is_a antigen processing and presentation of endogenous peptide antigen via MHC class I via ER pathway [GO:0002484]